{
  "term_label": "nucleus",
  "gene_symbol": "ZNF548",
  "term_id": "GO:0005634",
  "gene_name": "Zinc finger protein 548",
  "gene": "UniProtKB:Q8NEK5"
}